neuron projection arborization [GO:0140058] (biological process) References: PMID:17114044, PMID:23270857, PMID:23764288 Sources: GOC:aruk, GOC:bc Regulation: regulated by regulation of neuron projection arborization [GO:0150011]; RO_0002213 by GO:0150012; negatively regulated by negative regulation of neuron projection arborization [GO:0150013] Relationships: is a type of neuron projection morphogenesis [GO:0048812] Definition: The process in which the anatomical structures of a neuron projection are generated and organized into branches. A neuron projection is any process extending from a neural cell, such as axons or dendrites. Also known as: neurite arborization, neurite branching, neuron projection branching, branching morphogenesis of a neurite, branching morphogenesis of a neuron projection Subtypes: GO:0140059, axon arborization [GO:0140060]